{
  "term_label": "chromosome segregation",
  "gene_symbol": "TOP1",
  "term_id": "GO:0007059",
  "gene_name": "DNA topoisomerase 1",
  "gene": "UniProtKB:P11387"
}